endoplasmic reticulum protein-containing complex [GO:0140534] (cellular component) Subtypes: glycosylphosphatidylinositol-N-acetylglucosaminyltransferase (GPI-GnT) complex [GO:0000506], ER ubiquitin ligase complex [GO:0000835], GO:0005785, signal peptidase complex [GO:0005787], oligosaccharyltransferase complex [GO:0008250], GO:0009923, procollagen-proline 4-dioxygenase complex [GO:0016222], glucosidase II complex [GO:0017177], endoplasmic reticulum Sec complex [GO:0031205], Sec62/Sec63 complex [GO:0031207], endoplasmic reticulum palmitoyltransferase complex [GO:0031211], dolichyl-phosphate-mannose-protein mannosyltransferase complex [GO:0031502], ERMES complex [GO:0032865], SREBP-SCAP-Insig complex [GO:0032937], VCP-NPL4-UFD1 AAA ATPase complex [GO:0034098], luminal surveillance complex [GO:0034099], endoplasmic reticulum chaperone complex [GO:0034663], Ig heavy chain-bound endoplasmic reticulum chaperone complex [GO:0034664], GO:0036502, Derlin-1 retrotranslocation complex [GO:0036513], GO:0042765, MHC class I peptide loading complex [GO:0042824], TAP complex [GO:0042825], GET complex [GO:0043529], GO:0043541, GO:0061779, egasyn-beta-glucuronidase complex [GO:0070385], Dsl1/NZR complex [GO:0070939], translocon complex [GO:0071256], GO:0072546, mannosyl-oligosaccharide 1,2-alpha-mannosidase complex [GO:0106055], glycosylphosphatidylinositol-mannosyltransferase II complex [GO:0120097], GO:0160005, Ire1 complex [GO:1990332], ryanodine receptor complex [GO:1990425], glycosylphosphatidylinositol-mannosyltransferase I complex [GO:1990529], IRE1-TRAF2-ASK1 complex [GO:1990604], phospholamban complex [GO:1990629] Definition: A protein complex that is part of an endoplasmic reticulum. Relationships: is a type of protein-containing complex [GO:0032991]; is part of endoplasmic reticulum [GO:0005783] Sources: GOC:pg